{
  "gene": "UniProtKB:Q9NRD9",
  "term_id": "GO:0043020",
  "gene_name": "Dual oxidase 1",
  "gene_symbol": "DUOX1",
  "term_label": "NADPH oxidase complex"
}